{
  "gene_symbol": "CARTPT",
  "gene": "UniProtKB:Q16568",
  "term_label": "extracellular space",
  "term_id": "GO:0005615",
  "gene_name": "Cocaine- and amphetamine-regulated transcript protein"
}